{
  "term_id": "GO:0048477",
  "gene_symbol": "NANOS3",
  "term_label": "oogenesis",
  "gene_name": "Nanos homolog 3",
  "gene": "UniProtKB:P60323"
}